cellular response to hydroxyurea [GO:0072711] (biological process) Also known as: cellular response to HU Sources: GOC:mah Definition: Any process that results in a change in state or activity of a cell (in terms of movement, secretion, enzyme production, gene expression, etc.) as a result of a hydroxyurea stimulus. Relationships: is a type of response to hydroxyurea [GO:0072710]; is a type of cellular response to nitrogen compound [GO:1901699]